{
  "gene_symbol": "COX6C",
  "term_id": "GO:0005743",
  "term_label": "mitochondrial inner membrane",
  "gene": "UniProtKB:P09669",
  "gene_name": "Cytochrome c oxidase subunit 6C"
}